{
  "term_label": "'de novo' pyrimidine nucleobase biosynthetic process",
  "gene_symbol": "DHODH",
  "term_id": "GO:0006207",
  "gene": "UniProtKB:Q02127",
  "gene_name": "Dihydroorotate dehydrogenase (quinone), mitochondrial"
}